{
  "gene_symbol": "ANGPT1",
  "gene": "UniProtKB:Q15389",
  "term_id": "GO:0048014",
  "gene_name": "Angiopoietin-1",
  "term_label": "Tie signaling pathway"
}